purine nucleoside triphosphate catabolic process [GO:0009146] (biological process) Sources: GOC:go_curators, ISBN:0198506732 Also known as: purine nucleoside triphosphate breakdown, purine nucleoside triphosphate catabolism, purine nucleoside triphosphate degradation Relationships: is a type of nucleoside triphosphate catabolic process [GO:0009143]; is a type of purine nucleoside triphosphate metabolic process [GO:0009144] Subtypes: purine ribonucleoside triphosphate catabolic process [GO:0009207], purine deoxyribonucleoside triphosphate catabolic process [GO:0009217] Definition: The chemical reactions and pathways resulting in the breakdown of purine nucleoside triphosphate, a compound consisting of a purine base linked to a ribose or deoxyribose sugar esterified with triphosphate on the sugar.